P-body assembly [GO:0033962] (biological process) References: PMID:17429074 Sources: GOC:mah Also known as: P body assembly, cytoplasmic mRNA processing body assembly, P body biogenesis Relationships: is a type of membraneless organelle assembly [GO:0140694] Definition: The aggregation, arrangement and bonding together of proteins and RNA molecules to form a cytoplasmic mRNA processing body. Regulation: regulated by regulation of cytoplasmic mRNA processing body assembly [GO:0010603]; positively regulated by GO:0010606; negatively regulated by negative regulation of cytoplasmic mRNA processing body assembly [GO:0010607]